mucilage pectin biosynthetic process [GO:0048358] (biological process) Relationships: is a type of GO:0045489; is a type of mucilage pectin metabolic process [GO:0048363]; is part of GO:0010192 Sources: GOC:jid Definition: The chemical reactions and pathways resulting in the formation of the pectin component of mucilage. Also known as: mucilage pectin anabolism, mucilage pectin biosynthesis, mucilage pectin formation, mucilage pectin synthesis